regulation of sclerenchyma cell differentiation [GO:1904368] (biological process) References: PMID:26025534 Sources: GOC:TermGenie, GO_REF:0000058 Definition: Any process that modulates the frequency, rate or extent of sclerenchyma cell differentiation. Subtypes: GO:1904369 Relationships: is_a regulation of cell differentiation [GO:0045595]; RO_0002211 sclerenchyma cell differentiation [GO:0014001]